{
  "gene": "UniProtKB:D3DTV9",
  "gene_name": "Putative protein PRAC2",
  "gene_symbol": "PRAC2",
  "term_id": "UNKNOWN:0003",
  "term_label": "Unknown cellular component"
}